{
  "gene": "UniProtKB:O00167",
  "gene_symbol": "EYA2",
  "term_id": "GO:0030154",
  "gene_name": "Eyes absent homolog 2",
  "term_label": "cell differentiation"
}